15-cis-phytoene synthase activity [GO:0046905] (molecular function) Definition: Catalysis of the reaction: 2 geranylgeranyl diphosphate = 15-cis-phytoene + 2 diphosphate. Also known as: PSase activity, geranylgeranyl-diphosphate geranylgeranyltransferase activity, geranylgeranyl-diphosphate:geranylgeranyl-diphosphate geranylgeranyltransferase (15-cis-phytoene-forming) activity, phytoene synthase activity, prephytoene-diphosphate synthase activity Relationships: is a type of GO:0004659; is part of carotene biosynthetic process [GO:0016120] References: PMID:12641468 Sources: RHEA:34475